{
  "term_label": "Unknown biological process",
  "gene": "UniProtKB:Q8NFZ6",
  "term_id": "UNKNOWN:0002",
  "gene_symbol": "VN1R2",
  "gene_name": "Vomeronasal type-1 receptor 2"
}